cranial nerve development [GO:0021545] (biological process) Subtypes: GO:0021553, optic nerve development [GO:0021554], oculomotor nerve development [GO:0021557], trochlear nerve development [GO:0021558], trigeminal nerve development [GO:0021559], abducens nerve development [GO:0021560], facial nerve development [GO:0021561], vestibulocochlear nerve development [GO:0021562], glossopharyngeal nerve development [GO:0021563], GO:0021564, accessory nerve development [GO:0021565], hypoglossal nerve development [GO:0021566], lateral line nerve development [GO:0048892] Sources: GOC:cls, GOC:dgh, GOC:dph, GOC:jid, GO_REF:0000021 Relationships: is_a nerve development [GO:0021675] Definition: The process whose specific outcome is the progression of the cranial nerves over time, from its formation to the mature structure. The cranial nerves are composed of twelve pairs of nerves that emanate from the nervous tissue of the hindbrain. These nerves are sensory, motor, or mixed in nature, and provide the motor and general sensory innervation of the head, neck and viscera. They mediate vision, hearing, olfaction and taste and carry the parasympathetic innervation of the autonomic ganglia that control visceral functions.